regulation of branching morphogenesis of a nerve [GO:2000172] (biological process) Definition: Any process that modulates the frequency, rate or extent of branching morphogenesis of a nerve. Sources: GOC:BHF Relationships: is a type of regulation of morphogenesis of a branching structure [GO:0060688]; regulates branching morphogenesis of a nerve [GO:0048755] Subtypes: positive regulation of branching morphogenesis of a nerve [GO:1905492], negative regulation of branching morphogenesis of a nerve [GO:2000173]